{
  "gene": "UniProtKB:Q8N4G2",
  "term_label": "vesicle-mediated transport",
  "term_id": "GO:0016192",
  "gene_name": "ADP-ribosylation factor-like protein 14",
  "gene_symbol": "ARL14"
}